positive regulation of interleukin-20 production [GO:0032744] (BP) Definition: Any process that activates or increases the frequency, rate, or extent of interleukin-20 production. Sources: GOC:mah Also known as: positive regulation of IL-20 production, up regulation of interleukin-20 production, up-regulation of interleukin-20 production, upregulation of interleukin-20 production, activation of interleukin-20 production, positive regulation of interleukin-20 biosynthetic process, stimulation of interleukin-20 production Relationships: is a type of positive regulation of cytokine production [GO:0001819]; is a type of regulation of interleukin-20 production [GO:0032664]; RO_0002213 interleukin-20 production [GO:0032624]